{
  "gene_symbol": "PFN4",
  "gene_name": "Profilin-4",
  "term_id": "GO:0003785",
  "term_label": "actin monomer binding",
  "gene": "UniProtKB:Q8NHR9"
}